{
  "gene_symbol": "MYBPHL",
  "gene": "UniProtKB:A2RUH7",
  "term_id": "UNKNOWN:0003",
  "gene_name": "Myosin-binding protein H-like",
  "term_label": "Unknown cellular component"
}